{
  "gene_name": "Killer cell immunoglobulin-like receptor 2DL3",
  "term_label": "immune receptor activity",
  "gene_symbol": "KIR2DL3",
  "gene": "UniProtKB:P43628",
  "term_id": "GO:0140375"
}